anterior lateral line system development [GO:0048898] (BP) Definition: The process whose specific outcome is the progression of the anterior lateral line system over time, from its formation to the mature structure. The anterior lateral line system develops from cranial ectodermal placodes, situated between the eye and the ear, that give rise to both the neuromasts and the anterior lateral line sensory nerves that innervate the neuromasts. The anterior lateral line system consists of small sensory patches (neuromasts) located superficially on the skin or just under the skin in fluid-filled canals on the head of all fishes and most amphibians and are innervated by several lateral line nerves, which project to the hindbrain. The anterior lateral line system is stimulated by local water displacements and vibrations, and detects propulsion of the fish through the water, as well as facilitating shoaling, prey capture, and predator and obstacle avoidance. References: PMID:15018940 Sources: ISBN:0125296509 Relationships: is a type of lateral line system development [GO:0048925]; is part of mechanosensory lateral line system development [GO:0048881] Also known as: ALL system development